{
  "term_label": "Unknown biological process",
  "gene_name": "SH2 domain-containing protein 1A",
  "gene_symbol": "SH2D1A",
  "term_id": "UNKNOWN:0002",
  "gene": "UniProtKB:O60880"
}